{
  "term_label": "cardiac Troponin complex",
  "term_id": "GO:1990584",
  "gene": "UniProtKB:P63316",
  "gene_symbol": "TNNC1",
  "gene_name": "Troponin C, slow skeletal and cardiac muscles"
}